{
  "gene_name": "U4_U6 small nuclear ribonucleoprotein Prp31",
  "term_label": "Unknown molecular function",
  "term_id": "UNKNOWN:0001",
  "gene": "UniProtKB:Q8WWY3",
  "gene_symbol": "PRPF31"
}